RNA splicing, via transesterification reactions [GO:0000375] (biological process) Subtypes: RNA splicing, via transesterification reactions with guanosine as nucleophile [GO:0000376], GO:0000377 Also known as: RNA splicing factor activity, transesterification mechanism, pre-mRNA splicing factor activity, spliceosomal catalysis Sources: GOC:krc Note: Note that nuclear mRNA, Group I, Group II, and Group III introns are all spliced by a series of two transesterification reactions that occur within the RNA itself, or between two RNAs in trans splicing. Some of these require one or more proteins to stabilize the catalytic conformation, while others are autocatalytic. Note that tRNA introns are spliced by a different catalytic mechanism. Definition: Splicing of RNA via a series of two transesterification reactions. Relationships: is_a RNA splicing [GO:0008380]